mRNA transport [GO:0051028] (biological process) Definition: The directed movement of mRNA, messenger ribonucleic acid, into, out of or within a cell, or between cells, by means of some agent such as a transporter or pore. Sources: GOC:ai Relationships: is a type of RNA transport [GO:0050658] Subtypes: mRNA export from nucleus [GO:0006406]